ensheathment of neurons [GO:0007272] (biological process) Sources: GOC:dgh, GOC:dph, GOC:tb Relationships: is_a cellular process [GO:0009987]; is part of GO:0007399 Also known as: ionic insulation of neurons by glial cells Subtypes: axon ensheathment [GO:0008366], GO:0032295 Definition: The process in which glial cells envelop neuronal cell bodies and/or axons to form an insulating layer. This can take the form of myelinating or non-myelinating ensheathment.